{
  "term_label": "Unknown molecular function",
  "gene": "UniProtKB:A1E959",
  "gene_name": "Odontogenic ameloblast-associated protein",
  "gene_symbol": "ODAM",
  "term_id": "UNKNOWN:0001"
}